regulation of RNA biosynthetic process [GO:2001141] (biological process) Subtypes: regulation of DNA-templated transcription [GO:0006355], regulation of termination of DNA-templated transcription [GO:0031554], regulation of single stranded viral RNA replication via double stranded DNA intermediate [GO:0045091], regulation of promoter clearance from RNA polymerase II promoter [GO:0140845], GO:1902679, GO:1902680 Definition: Any process that modulates the frequency, rate or extent of RNA biosynthetic process. Sources: GOC:dph Also known as: regulation of RNA anabolism, regulation of RNA biosynthesis, regulation of RNA formation, regulation of RNA synthesis Relationships: is a type of regulation of macromolecule biosynthetic process [GO:0010556]; is a type of GO:0051252; regulates GO:0032774